negative regulation of norepinephrine uptake [GO:0051622] (biological process) Subtypes: inhibition of norepinephrine uptake [GO:0051624] Definition: Any process that stops, prevents, or reduces the frequency, rate or extent of the directed movement of norepinephrine into a cell. Also known as: down regulation of norepinephrine uptake, down-regulation of norepinephrine uptake, downregulation of norepinephrine uptake, negative regulation of levarterenol uptake, negative regulation of noradrenaline uptake, negative regulation of norepinephrine import Sources: GOC:ai Relationships: is a type of negative regulation of transport [GO:0051051]; is a type of regulation of norepinephrine uptake [GO:0051621]; negatively regulates norepinephrine uptake [GO:0051620]